{
  "gene_symbol": "DGCR8",
  "term_label": "microprocessor complex",
  "term_id": "GO:0070877",
  "gene": "UniProtKB:Q8WYQ5",
  "gene_name": "Microprocessor complex subunit DGCR8"
}